{
  "gene": "UniProtKB:Q9NYP9",
  "gene_name": "Protein Mis18-alpha",
  "term_label": "chromosome, centromeric region",
  "gene_symbol": "MIS18A",
  "term_id": "GO:0000775"
}